{
  "gene_symbol": "PDE6G",
  "term_label": "positive regulation of epidermal growth factor receptor signaling pathway",
  "gene_name": "Retinal rod rhodopsin-sensitive cGMP 3',5'-cyclic phosphodiesterase subunit gamma",
  "gene": "UniProtKB:P18545",
  "term_id": "GO:0045742"
}